{
  "gene_name": "ATP-binding cassette sub-family C member 4",
  "term_id": "GO:0016323",
  "gene_symbol": "ABCC4",
  "gene": "UniProtKB:O15439",
  "term_label": "basolateral plasma membrane"
}